mRNA alternative trans-splicing [GO:0000366] (biological process) Relationships: is a type of mRNA trans splicing, via spliceosome [GO:0000365]; is a type of GO:0000380 Also known as: intergenic mRNA trans splicing, intergenic nuclear mRNA trans splicing Definition: The joining together of two independently transcribed RNAs from two different genes, each of which also produces mRNA(s) via cis-splicing. References: PMID:11726664, PMID:12110900 Sources: GOC:krc